{
  "term_id": "GO:0005737",
  "gene_name": "Porphobilinogen deaminase",
  "term_label": "cytoplasm",
  "gene": "UniProtKB:P08397",
  "gene_symbol": "HMBS"
}